{
  "gene": "UniProtKB:Q8WTU0",
  "term_id": "GO:0004190",
  "gene_name": "Protein DDI1 homolog 1",
  "term_label": "aspartic-type endopeptidase activity",
  "gene_symbol": "DDI1"
}